{
  "term_label": "myosin II complex",
  "gene_symbol": "MYH7B",
  "term_id": "GO:0016460",
  "gene_name": "Myosin-7B",
  "gene": "UniProtKB:A7E2Y1"
}